{
  "term_label": "plasma membrane",
  "term_id": "GO:0005886",
  "gene_name": "Prokineticin receptor 1",
  "gene": "UniProtKB:Q8TCW9",
  "gene_symbol": "PROKR1"
}